{
  "gene": "UniProtKB:O75541",
  "gene_symbol": "ZNF821",
  "gene_name": "Zinc finger protein 821",
  "term_label": "regulation of transcription by RNA polymerase II",
  "term_id": "GO:0006357"
}